dinoflagellate cingulum [GO:0097611] (cellular component) Definition: A cell surface furrow that wraps around a dinoflagellate cell; the transverse flagellum lies in it. Note: The term name refers to a taxonomic group to make the label unique with respect to similarly-named anatomical structures. Also known as: cingulum, girdle, transverse groove References: PMID:7002229 Sources: GOC:at, Wikipedia:Dinoflagellate#Morphology, http://tolweb.org/Dinoflagellates/2445 Relationships: is a type of cell surface furrow [GO:0097610]